{
  "gene_symbol": "ACO1",
  "term_label": "3 iron, 4 sulfur cluster binding",
  "gene": "UniProtKB:P21399",
  "term_id": "GO:0051538",
  "gene_name": "Cytoplasmic aconitate hydratase"
}